interleukin-18 binding [GO:0042007] (molecular function) Relationships: is a type of GO:0019955 Also known as: IL-18 binding Sources: GOC:jl Definition: Binding to interleukin-18.